{
  "term_label": "olfactory receptor activity",
  "gene_symbol": "OR2A25",
  "gene_name": "Olfactory receptor 2A25",
  "term_id": "GO:0004984",
  "gene": "UniProtKB:A4D2G3"
}